{
  "gene_name": "Charged multivesicular body protein 7",
  "gene": "UniProtKB:Q8WUX9",
  "term_label": "vesicle budding from membrane",
  "term_id": "GO:0006900",
  "gene_symbol": "CHMP7"
}